{
  "term_id": "GO:0031463",
  "term_label": "Cul3-RING ubiquitin ligase complex",
  "gene_name": "Kelch-like protein 26",
  "gene_symbol": "KLHL26",
  "gene": "UniProtKB:Q53HC5"
}